{
  "term_id": "UNKNOWN:0002",
  "gene_name": "EF-hand and coiled-coil domain-containing protein 1",
  "gene_symbol": "EFCC1",
  "gene": "UniProtKB:Q9HA90",
  "term_label": "Unknown biological process"
}